sterol 3-beta-glucosyltransferase activity [GO:0016906] (molecular function) Also known as: UDP-glucose:sterol glucosyltransferase activity, UDPG:sterol glucosyltransferase activity, sterol glucosyltransferase activity, sterol:UDPG glucosyltransferase activity, UDP-glucose-sterol beta-glucosyltransferase activity, UDP-glucose-sterol glucosyltransferase activity, UDP-glucose:sterol 3-O-beta-D-glucosyltransferase activity, UDPG-SGTase activity, UDPglucose:sterol 3-O-beta-D-glucosyltransferase activity, sterol 3beta-glucosyltransferase activity, sterol-beta-D-glucosyltransferase activity, uridine diphosphoglucose-poriferasterol glucosyltransferase activity, uridine diphosphoglucose-sterol glucosyltransferase activity Definition: Catalysis of the reaction: UDP-glucose + a sterol = UDP + an O-glucosylsterol. Relationships: is a type of UDP-glucosyltransferase activity [GO:0035251] Sources: EC:2.4.1.173, RHEA:22724